{
  "term_label": "exonucleolytic trimming to generate mature 3'-end of 5.8S rRNA from tricistronic rRNA transcript (SSU-rRNA, 5.8S rRNA, LSU-rRNA)",
  "gene_name": "ERI1 exoribonuclease 3",
  "gene_symbol": "ERI3",
  "gene": "UniProtKB:O43414",
  "term_id": "GO:0000467"
}